{
  "term_label": "TORC1 signaling",
  "term_id": "GO:0038202",
  "gene": "UniProtKB:Q8N122",
  "gene_symbol": "RPTOR",
  "gene_name": "Regulatory-associated protein of mTOR"
}